negative regulation of RNA export from nucleus [GO:0046832] (biological process) Subtypes: negative regulation of tRNA export from nucleus [GO:2000239] Also known as: down regulation of RNA export from nucleus, down-regulation of RNA export from nucleus, downregulation of RNA export from nucleus, negative regulation of RNA export from cell nucleus, negative regulation of RNA export out of nucleus, negative regulation of RNA transport from nucleus to cytoplasm, negative regulation of RNA-nucleus export, inhibition of RNA export from nucleus Sources: GOC:bf Relationships: is a type of negative regulation of nucleobase-containing compound transport [GO:0032240]; is a type of GO:0046823; is a type of GO:0046831; negatively regulates GO:0006405 Definition: Any process that stops, prevents, or reduces the frequency, rate or extent of the directed movement of RNA from the nucleus into the cytoplasm.